terpene biosynthetic process [GO:0046246] (biological process) Relationships: is a type of isoprenoid biosynthetic process [GO:0008299]; is a type of terpene metabolic process [GO:0042214]; is a type of hydrocarbon biosynthetic process [GO:0120251] Definition: The chemical reactions and pathways resulting in the formation of terpenes, any of a large group of hydrocarbons made up of isoprene units. Subtypes: GO:0016120, ent-kaurene biosynthetic process [GO:0033332], isoprene biosynthetic process [GO:0043612], GO:0043693, GO:0051504, GO:0051762, ent-pimara-8(14),15-diene biosynthetic process [GO:1901541], miltiradiene biosynthetic process [GO:1901946], sesquarterpene biosynthetic process [GO:1903193] Also known as: terpene anabolism, terpene biosynthesis, terpene formation, terpene synthesis Sources: GOC:ai